{
  "term_label": "Unknown cellular component",
  "gene": "UniProtKB:Q70JA7",
  "gene_symbol": "CHSY3",
  "gene_name": "Chondroitin sulfate synthase 3",
  "term_id": "UNKNOWN:0003"
}